{
  "term_id": "GO:0099530",
  "term_label": "G protein-coupled receptor activity involved in regulation of postsynaptic membrane potential",
  "gene_name": "Metabotropic glutamate receptor 5",
  "gene_symbol": "GRM5",
  "gene": "UniProtKB:P41594"
}